{
  "gene_symbol": "COL9A3",
  "gene": "UniProtKB:Q14050",
  "term_id": "GO:0030020",
  "term_label": "extracellular matrix structural constituent conferring tensile strength",
  "gene_name": "Collagen alpha-3(IX) chain"
}